positive regulation of filamentous growth of a population of unicellular organisms [GO:1900430] (biological process) Also known as: up regulation of filamentous growth of a population of unicellular organisms, up-regulation of filamentous growth of a population of unicellular organisms, upregulation of filamentous growth of a population of unicellular organisms, activation of filamentous growth of a population of unicellular organisms Relationships: is_a GO:0090033; is a type of GO:1900428; positively regulates GO:0044182 Sources: GOC:TermGenie, GOC:di Subtypes: positive regulation of growth of unicellular organism as a thread of attached cells [GO:0070786], positive regulation of filamentous growth of a population of unicellular organisms in response to heat [GO:1900433], GO:1900436, positive regulation of filamentous growth of a population of unicellular organisms in response to chemical stimulus [GO:1900439], positive regulation of filamentous growth of a population of unicellular organisms in response to biotic stimulus [GO:1900445], GO:1900743 Definition: Any process that activates or increases the frequency, rate or extent of filamentous growth of a population of unicellular organisms.